{
  "gene_symbol": "KIAA0040",
  "gene": "UniProtKB:Q15053",
  "term_label": "Unknown cellular component",
  "term_id": "UNKNOWN:0003",
  "gene_name": "Uncharacterized protein KIAA0040"
}